{
  "term_label": "nucleus",
  "gene": "UniProtKB:P49639",
  "term_id": "GO:0005634",
  "gene_name": "Homeobox protein Hox-A1",
  "gene_symbol": "HOXA1"
}